{
  "term_id": "UNKNOWN:0002",
  "gene_name": "Elongin-A",
  "term_label": "Unknown biological process",
  "gene": "UniProtKB:Q14241",
  "gene_symbol": "ELOA"
}